{
  "gene_name": "Dual oxidase maturation factor 1",
  "term_label": "membrane",
  "gene_symbol": "DUOXA1",
  "term_id": "GO:0016020",
  "gene": "UniProtKB:Q1HG43"
}